{
  "term_label": "chromosome organization involved in meiotic cell cycle",
  "gene_name": "DNA repair protein RAD50",
  "term_id": "GO:0070192",
  "gene": "UniProtKB:Q92878",
  "gene_symbol": "RAD50"
}